{
  "gene": "UniProtKB:Q08378",
  "gene_name": "Golgin subfamily A member 3",
  "term_id": "UNKNOWN:0002",
  "term_label": "Unknown biological process",
  "gene_symbol": "GOLGA3"
}